acetylcholine:proton antiporter activity [GO:0005278] (molecular function) Also known as: acetylcholine:hydrogen antiporter activity Relationships: is a type of acetylcholine transmembrane transporter activity [GO:0005277]; is a type of proton transmembrane transporter activity [GO:0015078]; is a type of antiporter activity [GO:0015297] Sources: TC:2.A.1.2.13 Definition: Enables the transfer of a solute or solutes from one side of a membrane to the other according to the reaction: H+(out) + acetylcholine(in) = H+(in) + acetylcholine(out).